{
  "gene_name": "Endoplasmic reticulum-Golgi intermediate compartment protein 3",
  "gene": "UniProtKB:Q9Y282",
  "term_id": "UNKNOWN:0001",
  "gene_symbol": "ERGIC3",
  "term_label": "Unknown molecular function"
}